{
  "gene_symbol": "RAD51AP2",
  "gene_name": "RAD51-associated protein 2",
  "term_label": "protein-containing complex",
  "term_id": "GO:0032991",
  "gene": "UniProtKB:Q09MP3"
}